{
  "gene": "UniProtKB:Q9Y6J6",
  "term_id": "GO:0097623",
  "gene_symbol": "KCNE2",
  "gene_name": "Potassium voltage-gated channel subfamily E member 2",
  "term_label": "potassium ion export across plasma membrane"
}